{
  "gene": "UniProtKB:Q4V339",
  "term_label": "zinc chaperone activity",
  "gene_symbol": "ZNG1F",
  "term_id": "GO:0140827",
  "gene_name": "Zinc-regulated GTPase metalloprotein activator 1F"
}